citrate catabolic process to diacetyl [GO:0019651] (biological process) Also known as: citrate fermentation to diacetyl, diacetyl fermentation Sources: MetaCyc:P126-PWY Definition: The anaerobic chemical reactions and pathways resulting in the breakdown of citrate to diacetyl, yielding energy in the form of ATP. Relationships: is a type of citrate metabolic process [GO:0006101]; is a type of GO:0019662; is a type of ketone metabolic process [GO:0042180]; is a type of tricarboxylic acid catabolic process [GO:0072352]